wing disc morphogenesis [GO:0007472] (biological process) Relationships: is a type of imaginal disc morphogenesis [GO:0007560]; BFO_0000050 wing disc development [GO:0035220] Also known as: wing disc metamorphosis Definition: The process in which the anatomical structures derived from the wing disc are generated and organized. This includes the transformation of a wing imaginal disc from a monolayered epithelium in the larvae of holometabolous insects into recognizable adult structures including the wing hinge, wing blade and pleura. Sources: GOC:bf, ISBN:0879694238